{
  "gene_name": "Voltage-dependent calcium channel gamma-4 subunit",
  "term_id": "GO:0016247",
  "term_label": "channel regulator activity",
  "gene": "UniProtKB:Q9UBN1",
  "gene_symbol": "CACNG4"
}